positive regulation of lymphocyte apoptotic process [GO:0070230] (biological process) Note: Note that a lymphocyte is a cell of the B cell, T cell, or natural killer cell lineage (CL:0000542). Sources: GOC:add, GOC:mtg_apoptosis, ISBN:0781765196 Relationships: is a type of regulation of lymphocyte apoptotic process [GO:0070228]; is a type of positive regulation of leukocyte apoptotic process [GO:2000108]; positively regulates lymphocyte apoptotic process [GO:0070227] Subtypes: positive regulation of B cell apoptotic process [GO:0002904], positive regulation of T cell apoptotic process [GO:0070234], positive regulation of natural killer cell apoptotic process [GO:0070249] Also known as: up regulation of lymphocyte apoptosis, up-regulation of lymphocyte apoptosis, upregulation of lymphocyte apoptosis, activation of lymphocyte apoptosis, positive regulation of lymphocyte apoptosis, stimulation of lymphocyte apoptosis Definition: Any process that activates or increases the frequency, rate or extent of lymphocyte death by apoptotic process.